{
  "gene_name": "Myosin-7B",
  "gene": "UniProtKB:A7E2Y1",
  "term_label": "microfilament motor activity",
  "term_id": "GO:0000146",
  "gene_symbol": "MYH7B"
}